cell proliferation involved in heart valve development [GO:2000793] (biological process) Definition: Any cell proliferation that is involved in heart valve development. Relationships: is a type of cell population proliferation [GO:0008283]; BFO_0000050 heart valve development [GO:0003170] Also known as: cell proliferation of cardiac valve development, cell proliferation of heart valve development Subtypes: GO:0003249 Sources: GOC:BHF